{
  "term_label": "G protein-coupled receptor activity",
  "gene": "UniProtKB:Q6QNK2",
  "gene_name": "Adhesion G-protein coupled receptor D1",
  "gene_symbol": "ADGRD1",
  "term_id": "GO:0004930"
}